{
  "gene": "UniProtKB:O95936",
  "term_label": "endodermal cell fate specification",
  "gene_name": "Eomesodermin homolog",
  "gene_symbol": "EOMES",
  "term_id": "GO:0001714"
}